{
  "gene": "UniProtKB:A8MWY0",
  "gene_name": "Endosome_lysosome-associated apoptosis and autophagy regulator family member 2",
  "term_label": "Unknown molecular function",
  "gene_symbol": "ELAPOR2",
  "term_id": "UNKNOWN:0001"
}